{
  "gene": "UniProtKB:Q6DN03",
  "gene_symbol": "H2BC20P",
  "term_id": "GO:0019731",
  "gene_name": "Putative histone H2B type 2-C",
  "term_label": "antibacterial humoral response"
}